{
  "term_label": "U2 snRNA binding",
  "gene_symbol": "SF3B3",
  "gene": "UniProtKB:Q15393",
  "term_id": "GO:0030620",
  "gene_name": "Splicing factor 3B subunit 3"
}